auxin polar transport [GO:0009926] (biological process) Relationships: is a type of auxin transport [GO:0060918] Sources: GOC:sm Regulation: RO_0002211 by GO:2000012 Definition: The unidirectional movement of auxin in the stem from tip to base along the vector of gravity or basipetally. Subtypes: GO:0010540, GO:0010541